{
  "term_id": "GO:0005794",
  "gene_symbol": "CAV2",
  "gene": "UniProtKB:P51636",
  "gene_name": "Caveolin-2",
  "term_label": "Golgi apparatus"
}